{
  "gene_name": "Zinc finger and BTB domain-containing protein 17",
  "gene_symbol": "ZBTB17",
  "gene": "UniProtKB:Q13105",
  "term_id": "GO:0002682",
  "term_label": "regulation of immune system process"
}